{
  "gene_name": "Dynein light chain 1, cytoplasmic",
  "term_id": "GO:0005868",
  "term_label": "cytoplasmic dynein complex",
  "gene_symbol": "DYNLL1",
  "gene": "UniProtKB:P63167"
}